{
  "gene_name": "Sortilin",
  "term_id": "GO:0016020",
  "gene": "UniProtKB:Q99523",
  "term_label": "membrane",
  "gene_symbol": "SORT1"
}